apocarotenoid catabolic process [GO:0043290] (biological process) Definition: The chemical reactions and pathways resulting in the breakdown of apocarotenoids, a class of compounds derived from the oxidative cleavage of carotenoids, many of which are biologically important e.g. retinal and abscisic acid. Subtypes: abscisic acid catabolic process [GO:0046345] Relationships: is_a isoprenoid catabolic process [GO:0008300] Also known as: apo carotenoid catabolic process, apocarotenoid breakdown, apocarotenoid catabolism, apocarotenoid degradation References: PMID:33721905, PMID:34956282 Sources: GOC:jl